yolk [GO:0060417] (cellular component) Definition: The cytoplasmic part that serves as a nutrient reserve or energy source for the developing embryo. Relationships: is a type of cellular anatomical structure [GO:0110165]; is part of cytoplasm [GO:0005737] References: PMID:18046696 Sources: GOC:dph, GOC:tb